{
  "gene": "UniProtKB:Q86W50",
  "term_label": "23S rRNA (adenine(1618)-N(6))-methyltransferase activity",
  "term_id": "GO:0052907",
  "gene_symbol": "METTL16",
  "gene_name": "RNA N6-adenosine-methyltransferase METTL16"
}